{
  "term_id": "GO:0030194",
  "term_label": "positive regulation of blood coagulation",
  "gene_name": "Proteinase-activated receptor 1",
  "gene": "UniProtKB:P25116",
  "gene_symbol": "F2R"
}